{
  "gene_symbol": "UCKL1",
  "term_label": "Unknown biological process",
  "gene_name": "Uridine-cytidine kinase-like 1",
  "gene": "UniProtKB:Q9NWZ5",
  "term_id": "UNKNOWN:0002"
}